{
  "term_id": "GO:0046486",
  "gene": "UniProtKB:P52824",
  "gene_name": "Diacylglycerol kinase theta",
  "gene_symbol": "DGKQ",
  "term_label": "glycerolipid metabolic process"
}